{
  "gene_name": "PHD finger protein 12",
  "term_label": "negative regulation of transcription by RNA polymerase II",
  "gene": "UniProtKB:Q96QT6",
  "gene_symbol": "PHF12",
  "term_id": "GO:0000122"
}